{
  "term_id": "UNKNOWN:0001",
  "gene_name": "Cytoskeleton-associated protein 2",
  "gene_symbol": "CKAP2",
  "term_label": "Unknown molecular function",
  "gene": "UniProtKB:Q8WWK9"
}